{
  "gene_name": "G-patch domain and KOW motifs-containing protein",
  "gene": "UniProtKB:Q92917",
  "gene_symbol": "GPKOW",
  "term_id": "GO:0005681",
  "term_label": "spliceosomal complex"
}